{
  "term_id": "GO:0006891",
  "gene_name": "Vesicle-fusing ATPase",
  "gene_symbol": "NSF",
  "gene": "UniProtKB:P46459",
  "term_label": "intra-Golgi vesicle-mediated transport"
}